methyl farnesoate epoxidase activity [GO:0120511] (molecular function) Also known as: CYP15A1 activity Relationships: is a type of GO:0016712 Definition: Catalysis of the reaction: methyl (2E,6E)-farnesoate + O2 + reduced [NADPH--hemoprotein reductase] = H+ + H2O + juvenile hormone III + oxidized [NADPH--hemoprotein reductase]. References: PMID:23586995, PMID:38741075 Sources: RHEA:43728